thiamine triphosphate phosphatase activity [GO:0050333] (molecular function) Also known as: ThTPase activity, thiamin-triphosphatase activity, thiamine triphosphatase activity, thiamine-triphosphatase activity, thiamine-triphosphate phosphohydrolase activity Definition: Catalysis of the reaction: H2O + thiamine triphosphate = thiamine diphosphate + H+ + phosphate. Sources: RHEA:11744 Relationships: is a type of pyrophosphatase activity [GO:0016462]